{
  "term_id": "UNKNOWN:0003",
  "gene": "UniProtKB:A0A2R9YJI8",
  "gene_symbol": "A0A2R9YJI8",
  "gene_name": "Uncharacterized protein",
  "term_label": "Unknown cellular component"
}